viral nucleocapsid [GO:0019013] (cellular component) Definition: The complete protein-nucleic acid complex that is the packaged form of the genome in a virus particle. Relationships: is a type of GO:0044423; is part of viral capsid [GO:0019028] Also known as: core, nucleocapsid Sources: ISBN:0781702534